establishment of left sidedness [GO:0061967] (BP) Sources: GOC:18629866, GOC:BHF Relationships: is a type of establishment of left/right asymmetry [GO:0061966] Definition: The initial formation of the type asymmetry in an organism's body plan or part of an organism that established the pattern characteristic to its left side.